B2 bradykinin receptor binding [GO:0031713] (molecular function) Sources: GOC:mah, GOC:nln Definition: Binding to a B2 bradykinin receptor. Also known as: B2 bradykinin receptor ligand Relationships: is_a GO:0031711